{
  "gene": "UniProtKB:P07498",
  "term_label": "protein stabilization",
  "gene_name": "Kappa-casein",
  "term_id": "GO:0050821",
  "gene_symbol": "CSN3"
}